{
  "term_label": "actin cytoskeleton organization",
  "gene_symbol": "WASF1",
  "gene": "UniProtKB:Q92558",
  "gene_name": "Actin-binding protein WASF1",
  "term_id": "GO:0030036"
}